{
  "term_id": "GO:0005634",
  "gene_symbol": "VAX1",
  "term_label": "nucleus",
  "gene_name": "Ventral anterior homeobox 1",
  "gene": "UniProtKB:Q5SQQ9"
}